regulation of protein insertion into mitochondrial outer membrane [GO:1903636] (biological process) References: PMID:16374546 Sources: GOC:TermGenie, GO_REF:0000058 Subtypes: negative regulation of protein insertion into mitochondrial outer membrane [GO:1903637], positive regulation of protein insertion into mitochondrial outer membrane [GO:1903638] Also known as: regulation of mitochondrial outer membrane protein import, regulation of protein import into mitochondrial outer membrane, regulation of protein transport into mitochondrial outer membrane Definition: Any process that modulates the frequency, rate or extent of protein insertion into mitochondrial outer membrane. Relationships: is a type of regulation of mitochondrion organization [GO:0010821]; is a type of regulation of cellular localization [GO:0060341]; is a type of GO:1903214; regulates protein insertion into mitochondrial outer membrane [GO:0045040]